erythrose-4-phosphate dehydrogenase activity [GO:0048001] (molecular function) Definition: Catalysis of the reaction: D-erythrose 4-phosphate + H2O + NAD+ = 4-phospho-D-erythronate + 2 H+ + NADH. Relationships: is a type of oxidoreductase activity, acting on the aldehyde or oxo group of donors, NAD or NADP as acceptor [GO:0016620] Sources: EC:1.2.1.72, RHEA:12056 Also known as: D-erythrose 4-phosphate:NAD+ oxidoreductase activity, E4P dehydrogenase activity, E4PDH, Epd dehydrogenase activity, GapB, erythrose 4-phosphate dehydrogenase activity